carbon fixation by acetyl-CoA pathway [GO:0030634] (BP) References: PMID:11607093 Also known as: Ljungdahl-Wood pathway, reductive acetyl CoA pathway, acetyl CoA pathway Definition: A pathway of carbon dioxide fixation in which one molecule of acetyl-CoA is completely synthesized from two molecules of carbon dioxide (CO2). Relationships: is a type of GO:0006085; is a type of carbon fixation [GO:0015977]